{
  "gene_name": "Putative ribosomal RNA-processing protein 7 homolog B",
  "term_id": "GO:0006364",
  "term_label": "rRNA processing",
  "gene_symbol": "RRP7BP",
  "gene": "UniProtKB:Q9NSQ0"
}